glycosylceramidase activity [GO:0017042] (molecular function) Subtypes: galactosylceramidase activity [GO:0004336], glucosylceramidase activity [GO:0004348] Also known as: cerebrosidase activity, glycosyl ceramide glycosylhydrolase activity, glycosyl-N-acylsphingosine glycohydrolase activity Relationships: is a type of hydrolase activity, hydrolyzing O-glycosyl compounds [GO:0004553] References: PMID:10692580, PMID:9762914 Sources: EC:3.2.1.62 Definition: Catalysis of the reaction: glycosyl-N-acylsphingosine + H2O = a sugar + N-acylsphingosine.